supramolecular fiber [GO:0099512] (cellular component) Relationships: is a type of supramolecular polymer [GO:0099081] Subtypes: microfibril [GO:0001527], myosin filament [GO:0032982], contractile muscle fiber [GO:0043292], GO:0061800, intranuclear rod [GO:0061836], elastic fiber [GO:0071953], cytoophidium [GO:0097268], collagen beaded filament [GO:0098647], polymeric cytoskeletal fiber [GO:0099513] Definition: A polymer consisting of an indefinite number of protein or protein complex subunits that have polymerised to form a fiber-shaped structure. Also known as: fibril Sources: GOC:dos